{
  "term_label": "centriole",
  "gene_symbol": "DEUP1",
  "gene": "UniProtKB:Q05D60",
  "gene_name": "Deuterosome assembly protein 1",
  "term_id": "GO:0005814"
}